{
  "gene_name": "Zinc finger protein 286A",
  "term_label": "DNA-binding transcription factor activity, RNA polymerase II-specific",
  "gene_symbol": "ZNF286A",
  "term_id": "GO:0000981",
  "gene": "UniProtKB:Q9HBT8"
}